{
  "gene_name": "Putative protein BCL8",
  "gene_symbol": "NBEAP1",
  "term_id": "UNKNOWN:0002",
  "term_label": "Unknown biological process",
  "gene": "UniProtKB:P0C6P0"
}